commitment of neuronal cell to specific neuron type in forebrain [GO:0021902] (biological process) Definition: The commitment of neuronal precursor cells to become specialized types of neurons in the forebrain. Relationships: is a type of forebrain neuron fate commitment [GO:0021877] References: PMID:16226447 Sources: GOC:cls, GOC:dgh, GOC:dph, GOC:jid, GO_REF:0000021